{
  "gene": "UniProtKB:Q9ULH4",
  "gene_name": "Leucine-rich repeat and fibronectin type-III domain-containing protein 2",
  "term_id": "UNKNOWN:0002",
  "gene_symbol": "LRFN2",
  "term_label": "Unknown biological process"
}